glioblast division [GO:0048860] (biological process) Subtypes: subpallium glioblast cell division [GO:0021850], pallium glioblast division [GO:0022016] Relationships: is a type of GO:0051301 Definition: The process resulting in the physical partitioning and separation of a glioblast into daughter cells. Sources: GOC:devbiol